{
  "term_label": "neuron projection",
  "gene": "UniProtKB:Q96M98",
  "gene_name": "Parkin coregulated gene protein",
  "term_id": "GO:0043005",
  "gene_symbol": "PACRG"
}